nitrate metabolic process [GO:0042126] (BP) Definition: The chemical reactions and pathways involving nitrates, inorganic or organic salts and esters of nitric acid. Sources: GOC:jl Also known as: nitrate metabolism Subtypes: nitrate assimilation [GO:0042128], nitrate catabolic process [GO:0043602] Relationships: is a type of oxoacid metabolic process [GO:0043436]; is a type of GO:2001057